{
  "term_label": "Prp19 complex",
  "gene": "UniProtKB:O75934",
  "gene_symbol": "BCAS2",
  "gene_name": "Pre-mRNA-splicing factor SPF27",
  "term_id": "GO:0000974"
}